{
  "gene_name": "Cylicin-1",
  "gene": "UniProtKB:P35663",
  "term_id": "UNKNOWN:0002",
  "gene_symbol": "CYLC1",
  "term_label": "Unknown biological process"
}